{
  "gene": "UniProtKB:P49585",
  "term_label": "choline-phosphate cytidylyltransferase activity",
  "gene_symbol": "PCYT1A",
  "term_id": "GO:0004105",
  "gene_name": "Choline-phosphate cytidylyltransferase A"
}